heterotetrameric ADPG pyrophosphorylase complex [GO:0030931] (cellular component) Definition: A protein complex composed of four different subunits that possesses ADPG pyrophosphorylase activity. An example of this process is found in Mus musculus. Sources: GOC:mah, GOC:mtg_sensu Relationships: is a type of GO:0030929 Subtypes: GO:0031009